{
  "gene_name": "Serine_threonine-protein kinase OSR1",
  "gene_symbol": "OXSR1",
  "term_label": "positive regulation of T cell chemotaxis",
  "gene": "UniProtKB:O95747",
  "term_id": "GO:0010820"
}